{
  "gene": "UniProtKB:Q9NS85",
  "gene_name": "Carbonic anhydrase-related protein 10",
  "term_id": "UNKNOWN:0002",
  "term_label": "Unknown biological process",
  "gene_symbol": "CA10"
}